{
  "gene_name": "Angiopoietin-related protein 3",
  "gene": "UniProtKB:Q9Y5C1",
  "term_label": "cholesterol homeostasis",
  "gene_symbol": "ANGPTL3",
  "term_id": "GO:0042632"
}